{
  "term_label": "Unknown molecular function",
  "gene_name": "Transmembrane protein 102",
  "gene_symbol": "TMEM102",
  "gene": "UniProtKB:Q8N9M5",
  "term_id": "UNKNOWN:0001"
}